GPI anchor binding [GO:0034235] (molecular function) Subtypes: lipoarabinomannan binding [GO:0001876] Note: Note that this term should be used to annotate gene products that interact non-covalently with GPI anchors, and not proteins that have GPI anchors covalently attached. Also known as: glycosylphosphatidylinositol binding Relationships: is a type of phosphatidylinositol binding [GO:0035091]; is a type of GO:0051861 Sources: GOC:vw Definition: Binding to a glycosylphosphatidylinositol anchor. GPI anchors serve to attach membrane proteins to the lipid bilayer of cell membranes.